{
  "gene_symbol": "HBA2",
  "term_id": "GO:0005833",
  "term_label": "hemoglobin complex",
  "gene_name": "Hemoglobin subunit alpha",
  "gene": "UniProtKB:P69905"
}